{
  "gene": "UniProtKB:P57053",
  "gene_symbol": "H2BC12L",
  "term_id": "GO:0000786",
  "gene_name": "Histone H2B type F-S",
  "term_label": "nucleosome"
}